{
  "gene_symbol": "TAF11L8",
  "term_label": "RNA polymerase II general transcription initiation factor activity",
  "gene_name": "TATA-box-binding protein-associated factor 11-like protein 8",
  "gene": "UniProtKB:P0DW13",
  "term_id": "GO:0016251"
}